adhesion to host cell via type IV pili [GO:0052001] (biological process) Definition: Attachment of bacterial clusters to the surface of the host in a type IV pili dependent manner. The host is defined as the larger of the organisms involved in a symbiotic interaction. Relationships: is a type of adhesion of symbiont to host cell [GO:0044650] Also known as: type IV pili-dependent localized adherence to host Sources: GOC:ml